{
  "gene": "UniProtKB:Q96F07",
  "term_label": "axon guidance",
  "gene_name": "Cytoplasmic FMR1-interacting protein 2",
  "gene_symbol": "CYFIP2",
  "term_id": "GO:0007411"
}